{
  "gene_name": "Serine_threonine-protein kinase PLK2",
  "term_label": "spindle pole",
  "gene": "UniProtKB:Q9NYY3",
  "term_id": "GO:0000922",
  "gene_symbol": "PLK2"
}